organic phosphonate catabolic process [GO:0019700] (biological process) Also known as: phosphonate breakdown, phosphonate catabolism, phosphonate degradation, organophosphonate catabolic process Relationships: is a type of catabolic process [GO:0009056]; is a type of organic phosphonate metabolic process [GO:0019634] Sources: GOC:js Definition: The chemical reactions and pathways resulting in the breakdown of phosphonates, any organic compound containing one or more C-PO(OH)2 or C-PO(OR)2 (with R=alkyl, aryl) groups. Catabolism of phosphonic acid itself, an inorganic compound without the biochemically relevant C-P bond, is not included.